{
  "gene_symbol": "CCNH",
  "gene_name": "Cyclin-H",
  "term_id": "GO:0005634",
  "term_label": "nucleus",
  "gene": "UniProtKB:P51946"
}